{
  "gene": "UniProtKB:Q9NUH8",
  "term_label": "mitochondrial membrane",
  "gene_name": "Transmembrane protein 14B",
  "term_id": "GO:0031966",
  "gene_symbol": "TMEM14B"
}